{
  "gene_symbol": "CCDC106",
  "gene_name": "Coiled-coil domain-containing protein 106",
  "gene": "UniProtKB:Q9BWC9",
  "term_id": "GO:0005654",
  "term_label": "nucleoplasm"
}